{
  "term_label": "Unknown cellular component",
  "term_id": "UNKNOWN:0003",
  "gene_symbol": "RTL3",
  "gene": "UniProtKB:Q8N8U3",
  "gene_name": "Retrotransposon Gag-like protein 3"
}